cellular response to red or far red light [GO:0071489] (biological process) Subtypes: GO:0010017, GO:0071490, cellular response to red light [GO:0071491] Relationships: is a type of GO:0009639; is a type of cellular response to light stimulus [GO:0071482] Definition: Any process that results in a change in state or activity of a cell (in terms of movement, secretion, enzyme production, gene expression, etc.) as a result of a red or far red light stimulus. Red light is electromagnetic radiation of wavelength of 580-700nm. Far red light is electromagnetic radiation of wavelength 700-800nm. An example of this response is seen at the beginning of many plant species developmental stages. These include germination, and the point when cotyledon expansion is triggered. In certain species these processes take place in response to absorption of red light by the pigment molecule phytochrome, but the signal can be reversed by exposure to far red light. During the initial phase the phytochrome molecule is only present in the red light absorbing form, but on absorption of red light it changes to a far red light absorbing form, triggering progress through development. An immediate short period of exposure to far red light entirely returns the pigment to its initial state and prevents triggering of the developmental process. A thirty minute break between red and subsequent far red light exposure renders the red light effect irreversible, and development then occurs regardless of whether far red light exposure subsequently occurs. Sources: GOC:mah